{
  "term_label": "mRNA 3'-UTR binding",
  "gene": "UniProtKB:Q9BX46",
  "gene_name": "RNA-binding protein 24",
  "term_id": "GO:0003730",
  "gene_symbol": "RBM24"
}